{
  "gene_name": "EF-hand calcium-binding domain-containing protein 9",
  "term_label": "cytoplasm",
  "gene": "UniProtKB:A8MZ26",
  "gene_symbol": "EFCAB9",
  "term_id": "GO:0005737"
}